{
  "term_label": "GTPase activity",
  "gene_name": "EF-hand calcium-binding domain-containing protein 4B",
  "gene": "UniProtKB:Q9BSW2",
  "term_id": "GO:0003924",
  "gene_symbol": "CRACR2A"
}